inorganic ion homeostasis [GO:0098771] (biological process) Definition: Any process involved in the maintenance of an internal steady state of inorganic ions within an organism or cell. Sources: GOC:dos Relationships: is a type of chemical homeostasis [GO:0048878] Subtypes: GO:0006877, intracellular iron ion homeostasis [GO:0006879], intracellular zinc ion homeostasis [GO:0006882], magnesium ion homeostasis [GO:0010960], intracellular nickel ion homeostasis [GO:0035785], phosphate ion homeostasis [GO:0055062], sulfate ion homeostasis [GO:0055063], chloride ion homeostasis [GO:0055064], copper ion homeostasis [GO:0055070], manganese ion homeostasis [GO:0055071], calcium ion homeostasis [GO:0055074], potassium ion homeostasis [GO:0055075], sodium ion homeostasis [GO:0055078], multicellular organismal-level iron ion homeostasis [GO:0060586], GO:0097272, intracellular borate homeostasis [GO:0160070]